{
  "term_label": "serine-type endopeptidase activity",
  "gene_symbol": "PRSS3",
  "term_id": "GO:0004252",
  "gene": "UniProtKB:P35030",
  "gene_name": "Trypsin-3"
}